{
  "term_id": "GO:0000981",
  "gene_symbol": "IRX3",
  "gene": "UniProtKB:P78415",
  "gene_name": "Iroquois-class homeodomain protein IRX-3",
  "term_label": "DNA-binding transcription factor activity, RNA polymerase II-specific"
}